protein localization to pericentric heterochromatin [GO:1902682] (biological process) References: PMID:20211136 Sources: GOC:TermGenie, GO_REF:0000087 Definition: A process in which a protein is transported to, or maintained in the pericentric heterochromatin. Relationships: is a type of protein localization to chromosome, centromeric region [GO:0071459]; is a type of GO:0097355 Also known as: protein localisation in centromeric heterochromatin